{
  "term_label": "extracellular matrix organization",
  "term_id": "GO:0030198",
  "gene_name": "Uncharacterized protein C6orf15",
  "gene": "UniProtKB:Q6UXA7",
  "gene_symbol": "C6orf15"
}